{
  "term_label": "Unknown molecular function",
  "gene": "UniProtKB:Q9BU79",
  "gene_symbol": "TMEM243",
  "gene_name": "Transmembrane protein 243",
  "term_id": "UNKNOWN:0001"
}